activin receptor complex [GO:0048179] (cellular component) References: PMID:8307945, PMID:8622651 Definition: A protein complex that acts as an activin receptor. Heterodimeric activin receptors, comprising one Type I activin receptor and one Type II receptor polypeptide, and heterotrimeric receptors have been observed. Relationships: is a type of plasma membrane signaling receptor complex [GO:0098802]; is a type of serine/threonine protein kinase complex [GO:1902554]